{
  "term_label": "cytoplasm",
  "gene_name": "Diphosphoinositol polyphosphate phosphohydrolase NUDT4B",
  "gene_symbol": "NUDT4B",
  "gene": "UniProtKB:A0A024RBG1",
  "term_id": "GO:0005737"
}